{
  "term_label": "Unknown cellular component",
  "gene": "UniProtKB:Q9NRI6",
  "gene_symbol": "PYY2",
  "gene_name": "Putative peptide YY-2",
  "term_id": "UNKNOWN:0003"
}